{
  "term_label": "cytidine deaminase activity",
  "gene": "UniProtKB:Q8IUX4",
  "gene_symbol": "APOBEC3F",
  "gene_name": "DNA dC-dU-editing enzyme APOBEC-3F",
  "term_id": "GO:0004126"
}